{
  "gene_name": "Putative UPF0607 protein ENSP00000381514",
  "term_id": "UNKNOWN:0002",
  "gene_symbol": "A8MUA0",
  "gene": "UniProtKB:A8MUA0",
  "term_label": "Unknown biological process"
}